{
  "term_label": "postsynaptic membrane",
  "gene_symbol": "KCND3",
  "term_id": "GO:0045211",
  "gene_name": "Potassium voltage-gated channel subfamily D member 3",
  "gene": "UniProtKB:Q9UK17"
}